regulation of interleukin-24 production [GO:0032668] (biological process) Also known as: regulation of IL-24 production, regulation of interleukin-24 biosynthetic process Relationships: is a type of GO:0001817; RO_0002211 GO:0032628 Sources: GOC:mah Subtypes: GO:0032708, positive regulation of interleukin-24 production [GO:0032748] Definition: Any process that modulates the frequency, rate, or extent of interleukin-24 production.